{
  "gene": "UniProtKB:P14927",
  "term_label": "Unknown molecular function",
  "gene_symbol": "UQCRB",
  "term_id": "UNKNOWN:0001",
  "gene_name": "Cytochrome b-c1 complex subunit 7"
}